menaquinone-dependent protoporphyrinogen oxidase activity [GO:0070819] (molecular function) Definition: Catalysis of the reaction: protoporphyrinogen IX + menaquinone = protoporphyrin IX + reduced menaquinone. Relationships: is a type of oxidoreductase activity, acting on the CH-CH group of donors, quinone or related compound as acceptor [GO:0016635]; is a type of GO:0070818 References: PMID:19583219 Sources: GOC:mah Also known as: protoporphyrinogen-IX:menaquinone oxidoreductase activity